{
  "gene_symbol": "SMIM40",
  "gene": "UniProtKB:Q5STR5",
  "term_id": "UNKNOWN:0002",
  "term_label": "Unknown biological process",
  "gene_name": "Small integral membrane protein 40"
}